propionate metabolic process, methylcitrate cycle [GO:0019679] (biological process) Sources: GOC:go_curators Relationships: is a type of propionate metabolic process [GO:0019541] Definition: The chemical reactions and pathways involving propionate that occur in the methylcitrate cycle. Also known as: propionate metabolism, methylcitrate cycle